{
  "gene": "UniProtKB:P0CG34",
  "term_id": "GO:0031941",
  "gene_name": "Thymosin beta-15A",
  "term_label": "filamentous actin",
  "gene_symbol": "TMSB15A"
}